{
  "term_label": "Unknown cellular component",
  "term_id": "UNKNOWN:0003",
  "gene_symbol": "DELEC1",
  "gene": "UniProtKB:Q9P2X7",
  "gene_name": "Deleted in esophageal cancer 1"
}